negative regulation of peptide hormone processing [GO:0060570] (biological process) Definition: Any process that decreases the rate, frequency or extent of peptide hormone processing. Peptide hormone processing is the generation of a mature peptide hormone by posttranslational processing of a prohormone. Relationships: is a type of negative regulation of protein processing [GO:0010955]; is a type of negative regulation of hormone metabolic process [GO:0032351]; is a type of GO:0034249; is a type of regulation of peptide hormone processing [GO:0060568]; negatively regulates peptide hormone processing [GO:0016486] Sources: GOC:dph, GOC:tb